meiotic sister chromatid cohesion [GO:0051177] (biological process) Definition: The cell cycle process in which sister chromatids of a replicated chromosome are joined along the entire length of the chromosome during meiosis. Relationships: is a type of sister chromatid cohesion [GO:0007062] Sources: GOC:ai Subtypes: male meiosis sister chromatid cohesion [GO:0007065], female meiosis sister chromatid cohesion [GO:0007066], meiotic sister chromatid cohesion involved in meiosis I [GO:0010789], meiotic sister chromatid cohesion involved in meiosis II [GO:0010790], GO:0051754